{
  "term_id": "UNKNOWN:0003",
  "gene": "UniProtKB:O43934",
  "gene_name": "UNC93-like protein MFSD11",
  "gene_symbol": "MFSD11",
  "term_label": "Unknown cellular component"
}